{
  "term_label": "brain development",
  "gene_symbol": "VCX3B",
  "term_id": "GO:0007420",
  "gene_name": "Variable charge X-linked protein 3B",
  "gene": "UniProtKB:Q9H321"
}